{
  "gene_symbol": "DDX43",
  "term_label": "Unknown cellular component",
  "gene_name": "Probable ATP-dependent RNA helicase DDX43",
  "term_id": "UNKNOWN:0003",
  "gene": "UniProtKB:Q9NXZ2"
}